{
  "gene": "UniProtKB:Q13596",
  "gene_name": "Sorting nexin-1",
  "term_id": "GO:0035091",
  "term_label": "phosphatidylinositol binding",
  "gene_symbol": "SNX1"
}